stomach neuroendocrine cell differentiation [GO:0061102] (biological process) Also known as: gastric neuroendocrine cell differentiation Definition: The process in which a relatively unspecialized cell acquires specialized features of a neuroendocrine cell of the stomach epithelium. References: PMID:18173746 Sources: GOC:dph Regulation: RO_0002211 by regulation of stomach neuroendocrine cell differentiation [GO:0061105]; negatively regulated by GO:0061106 Relationships: is a type of enteroendocrine cell differentiation [GO:0035883]; is a type of neuroendocrine cell differentiation [GO:0061101]; is part of stomach development [GO:0062094]